{
  "term_label": "positive regulation of JNK cascade",
  "gene": "UniProtKB:P56706",
  "gene_name": "Protein Wnt-7b",
  "term_id": "GO:0046330",
  "gene_symbol": "WNT7B"
}